peptidyl-valine modification [GO:0018213] (biological process) Relationships: is a type of peptidyl-amino acid modification [GO:0018193] Definition: The modification of peptidyl-valine. Sources: GOC:go_curators